{
  "gene_symbol": "PLCB4",
  "gene_name": "1-phosphatidylinositol 4,5-bisphosphate phosphodiesterase beta-4",
  "term_label": "phosphatidylinositol-4,5-bisphosphate phospholipase C activity",
  "gene": "UniProtKB:Q15147",
  "term_id": "GO:0004435"
}